{
  "term_label": "Unknown molecular function",
  "gene": "UniProtKB:Q7Z422",
  "gene_name": "SUZ domain-containing protein 1",
  "gene_symbol": "SZRD1",
  "term_id": "UNKNOWN:0001"
}